{
  "term_id": "UNKNOWN:0001",
  "gene_symbol": "NTN4",
  "term_label": "Unknown molecular function",
  "gene": "UniProtKB:Q9HB63",
  "gene_name": "Netrin-4"
}